insulin-like growth factor I binding [GO:0031994] (molecular function) Relationships: is a type of GO:0005520 Definition: Binding to insulin-like growth factor I. Sources: GOC:mah Also known as: IGF-I binding